{
  "gene_symbol": "MRLN",
  "term_id": "UNKNOWN:0003",
  "term_label": "Unknown cellular component",
  "gene_name": "Myoregulin",
  "gene": "UniProtKB:P0DMT0"
}